{
  "term_id": "GO:0006376",
  "gene_symbol": "LUC7L2",
  "term_label": "mRNA splice site recognition",
  "gene": "UniProtKB:Q9Y383",
  "gene_name": "Putative RNA-binding protein Luc7-like 2"
}